regulation of cell fate specification [GO:0042659] (biological process) Definition: Any process that mediates the adoption of a specific fate by a cell. Sources: GOC:go_curators Relationships: is a type of regulation of cell fate commitment [GO:0010453]; regulates cell fate specification [GO:0001708] Subtypes: GO:0009996, regulation of atrichoblast fate specification [GO:0010058], regulation of trichoblast fate specification [GO:0010061], positive regulation of cell fate specification [GO:0042660], GO:0042661, regulation of endodermal cell fate specification [GO:0042663], GO:0042665, regulation of inner ear auditory receptor cell fate specification [GO:0042669], regulation of retinal cone cell fate specification [GO:0042673], regulation of compound eye cone cell fate specification [GO:0042682], regulation of neural crest cell fate specification [GO:1905295], regulation of cardiac cell fate specification [GO:2000043]